5-hydroxypentanoate CoA-transferase activity [GO:0047591] (molecular function) Also known as: 5-hydroxyvalerate CoA-transferase activity, 5-hydroxyvalerate coenzyme A transferase activity, acetyl-CoA:5-hydroxypentanoate CoA-transferase activity Relationships: is a type of CoA-transferase activity [GO:0008410] Sources: EC:2.8.3.14, RHEA:23496 Definition: Catalysis of the reaction: 5-hydroxypentanoate + acetyl-CoA = 5-hydroxy-pentanoyl-CoA + acetate.